{
  "gene": "UniProtKB:Q9HB55",
  "term_label": "testosterone 6-beta-hydroxylase activity",
  "gene_symbol": "CYP3A43",
  "term_id": "GO:0050649",
  "gene_name": "Cytochrome P450 3A43"
}